sno(s)RNA catabolic process [GO:0016077] (biological process) Also known as: sno(s)RNA breakdown, sno(s)RNA catabolism, sno(s)RNA degradation, sRNA catabolic process, snoRNA catabolic process Definition: The chemical reactions and pathways resulting in the breakdown of snoRNA, small nucleolar RNA, any of a class of small RNAs that are associated with the eukaryotic nucleus as components of small nucleolar ribonucleoproteins. Subtypes: GO:0071036 Relationships: is a type of GO:0006401; is a type of sno(s)RNA metabolic process [GO:0016074] Sources: GOC:krc, ISBN:0198506732